{
  "gene_symbol": "MEIS3",
  "gene": "UniProtKB:Q99687",
  "term_label": "angiogenesis",
  "gene_name": "Homeobox protein Meis3",
  "term_id": "GO:0001525"
}